{
  "term_id": "UNKNOWN:0003",
  "gene": "UniProtKB:Q9Y570",
  "term_label": "Unknown cellular component",
  "gene_symbol": "PPME1",
  "gene_name": "Protein phosphatase methylesterase 1"
}